{
  "term_label": "Unknown cellular component",
  "gene_symbol": "RASSF6",
  "term_id": "UNKNOWN:0003",
  "gene": "UniProtKB:Q6ZTQ3",
  "gene_name": "Ras association domain-containing protein 6"
}